{
  "gene_name": "Podocin",
  "term_label": "plasma membrane",
  "gene_symbol": "NPHS2",
  "gene": "UniProtKB:Q9NP85",
  "term_id": "GO:0005886"
}